SMN complex [GO:0032797] (cellular component) References: PMID:16434402, PMID:17023415 Definition: A protein complex that contains the survival motor neuron (SMN) protein and at least eight additional integral components, including the Gemin2-8 and Unrip proteins; the complex is found in the cytoplasm and in nuclear Gems, and is involved in spliceosomal snRNP assembly in the cytoplasm and in pre-mRNA splicing in the nucleus. Also known as: SMN core complex, survival motor neuron complex Relationships: is a type of Sm-like protein family complex [GO:0120114]; is part of GO:0034719 Note: Note that a larger complex containing Sm proteins and other subunits is also sometimes referred to as the 'SMN complex'. The larger complex is represented by 'SMN-Sm protein complex ; GO:0034719'.